{
  "term_id": "GO:0005789",
  "gene": "UniProtKB:P56937",
  "term_label": "endoplasmic reticulum membrane",
  "gene_symbol": "HSD17B7",
  "gene_name": "3-keto-steroid reductase_17-beta-hydroxysteroid dehydrogenase 7"
}